{
  "term_id": "GO:0005737",
  "gene_name": "Caprin-2",
  "term_label": "cytoplasm",
  "gene_symbol": "CAPRIN2",
  "gene": "UniProtKB:Q6IMN6"
}